{
  "gene": "UniProtKB:Q9UNI1",
  "gene_symbol": "CELA1",
  "term_id": "GO:0006508",
  "term_label": "proteolysis",
  "gene_name": "Chymotrypsin-like elastase family member 1"
}